anaphase-promoting complex-dependent catabolic process [GO:0031145] (biological process) Relationships: is a type of proteasome-mediated ubiquitin-dependent protein catabolic process [GO:0043161] Definition: The chemical reactions and pathways resulting in the breakdown of a protein or peptide by hydrolysis of its peptide bonds, initiated by the covalent attachment of ubiquitin, with ubiquitin-protein ligation catalyzed by the anaphase-promoting complex, and mediated by the proteasome. References: PMID:15380083, PMID:15840442 Sources: GOC:mah Regulation: regulated by regulation of anaphase-promoting complex-dependent catabolic process [GO:1905784]; negatively regulated by negative regulation of anaphase-promoting complex-dependent catabolic process [GO:1905785]; positively regulated by positive regulation of anaphase-promoting complex-dependent catabolic process [GO:1905786] Also known as: APC-dependent proteasomal ubiquitin-dependent protein catabolic process, APC-dependent proteasomal ubiquitin-dependent protein catabolism, anaphase-promoting complex-dependent proteasomal ubiquitin-dependent protein breakdown, anaphase-promoting complex-dependent proteasomal ubiquitin-dependent protein catabolic process, anaphase-promoting complex-dependent proteasomal ubiquitin-dependent protein catabolism, anaphase-promoting complex-dependent proteasomal ubiquitin-dependent protein degradation, cyclin breakdown, cyclin catabolic process, cyclin catabolism, cyclin degradation, degradation of cyclin, negative regulation of cyclin-dependent protein serine/threonine kinase by cyclin degradation